{
  "gene": "UniProtKB:P25440",
  "term_id": "GO:0005634",
  "gene_symbol": "BRD2",
  "gene_name": "Bromodomain-containing protein 2",
  "term_label": "nucleus"
}